Pho85-Pho80 CDK-cyclin complex [GO:1990860] (CC) Definition: A cyclin dependent kinase (CDK) complex that contains a kinase subunit and a regulatory cyclin subunit. An example of this complex in budding yeast S. cerevisiae consists of the Pho85 kinase and the Pho80 cyclin. References: PMID:8108735 Sources: GOC:rb Relationships: is a type of cyclin-dependent protein kinase holoenzyme complex [GO:0000307]